{
  "gene_symbol": "MAP3K11",
  "term_id": "GO:0005737",
  "gene_name": "Mitogen-activated protein kinase kinase kinase 11",
  "gene": "UniProtKB:Q16584",
  "term_label": "cytoplasm"
}